icosanoid transmembrane transporter activity [GO:0071714] (MF) Definition: Enables the transfer of icosanoids from one side of a membrane to the other. Relationships: is a type of lipid transmembrane transporter activity [GO:0170055]; BFO_0000050 icosanoid transport [GO:0071715] Sources: GOC:sl Also known as: eicosanoid transmembrane transporter activity Subtypes: prostaglandin transmembrane transporter activity [GO:0015132]